{
  "term_label": "killing of cells of another organism",
  "gene_symbol": "HTN3",
  "term_id": "GO:0031640",
  "gene_name": "Histatin-3",
  "gene": "UniProtKB:P15516"
}